discadenine biosynthetic process [GO:0034268] (biological process) Sources: GOC:mah Definition: The chemical reactions and pathways resulting in the formation of discadenine, (2S)-2-amino-4-{6-[(3-methylbut-2-en-1-yl)amino]-3H-purin-3-yl}butanoic acid. Also known as: discadenine anabolism, discadenine biosynthesis, discadenine formation, discadenine synthesis Relationships: is a type of cytokinin biosynthetic process [GO:0009691]; is a type of purine-containing compound biosynthetic process [GO:0072522]; is a type of L-amino acid biosynthetic process [GO:0170034]; is a type of non-proteinogenic amino acid biosynthetic process [GO:0170043]